positive regulation of postsynaptic density organization [GO:1905876] (biological process) Also known as: positive regulation of PSD organization, positive regulation of post synaptic density organization, positive regulation of post-synaptic density organization, positive regulation of postsynaptic density organisation, up regulation of PSD organization, up regulation of post synaptic density organization, up regulation of post-synaptic density organization, up regulation of postsynaptic density organisation, up regulation of postsynaptic density organization, up-regulation of PSD organization, up-regulation of post synaptic density organization, up-regulation of post-synaptic density organization, up-regulation of postsynaptic density organisation, up-regulation of postsynaptic density organization, upregulation of PSD organization, upregulation of post synaptic density organization, upregulation of post-synaptic density organization, upregulation of postsynaptic density organisation, upregulation of postsynaptic density organization, activation of PSD organization, activation of post synaptic density organization, activation of post-synaptic density organization, activation of postsynaptic density organisation, activation of postsynaptic density organization Definition: Any process that activates or increases the frequency, rate or extent of postsynaptic density organization. Relationships: is a type of positive regulation of organelle organization [GO:0010638]; is a type of GO:1905874; positively regulates postsynaptic density organization [GO:0097106] References: PMID:21887379 Sources: GOC:TermGenie, GO_REF:0000058 Subtypes: positive regulation of postsynaptic density assembly [GO:0160036]